{
  "gene_symbol": "OR4M2B",
  "term_label": "Unknown biological process",
  "term_id": "UNKNOWN:0002",
  "gene_name": "Olfactory receptor 4M2",
  "gene": "UniProtKB:A0A0X1KG70"
}